{
  "gene": "UniProtKB:P22492",
  "term_label": "double-stranded DNA binding",
  "gene_name": "Histone H1t",
  "gene_symbol": "H1-6",
  "term_id": "GO:0003690"
}